{
  "gene_name": "Putative methyltransferase C9orf114",
  "term_id": "GO:0031616",
  "term_label": "spindle pole centrosome",
  "gene": "UniProtKB:Q5T280",
  "gene_symbol": "SPOUT1"
}